{
  "term_label": "Unknown molecular function",
  "gene": "UniProtKB:Q68CZ2",
  "gene_name": "Tensin-3",
  "gene_symbol": "TNS3",
  "term_id": "UNKNOWN:0001"
}